{
  "gene": "UniProtKB:Q8WZ94",
  "term_id": "UNKNOWN:0003",
  "term_label": "Unknown cellular component",
  "gene_name": "Olfactory receptor 5P3",
  "gene_symbol": "OR5P3"
}